exosome (RNase complex) [GO:0000178] (CC) Note: Note that this term should not be confused with 'exosome' used in the context of vesicles released from multivesicular bodies. Definition: A ribonuclease complex that has 3-prime to 5-prime exoribonuclease activity and possibly endoribonuclease activity, producing 5-prime-phosphomonoesters. Participates in a multitude of cellular RNA processing and degradation events preventing nuclear export and/or translation of aberrant RNAs. Restricted to processing linear and circular single-stranded RNAs (ssRNA) only. RNAs with complex secondary structures may have to be unwound or pre-processed by co-factors prior to entering the complex, esp if the 3-prime end is structured. Also known as: exosome (ribonucleasease complex), exosome multienzyme ribonuclease complex References: PMID:17174896, PMID:20531386, PMID:26726035 Subtypes: nuclear exosome (RNase complex) [GO:0000176], cytoplasmic exosome (RNase complex) [GO:0000177] Relationships: is a type of exoribonuclease complex [GO:1905354]; is part of GO:0005622